{
  "gene_name": "Histone H2B type 2-K1",
  "term_id": "GO:0006325",
  "term_label": "chromatin organization",
  "gene_symbol": "H2BK1",
  "gene": "UniProtKB:A0A2R8Y619"
}